cell communication by chemical coupling [GO:0010643] (biological process) Definition: The process that mediates signaling interactions between one cell and another cell by the transfer of small, water-soluble molecules or metabolites between their adjacent cytoplasms via intercellular protein channels. Sources: GOC:dph, GOC:kmv, GOC:tb Relationships: is a type of cell communication [GO:0007154] Regulation: regulated by regulation of cell communication by chemical coupling [GO:0010645]; positively regulated by positive regulation of cell communication by chemical coupling [GO:0010652]; negatively regulated by negative regulation of cell communication by chemical coupling [GO:0010653]